{
  "gene": "UniProtKB:P54750",
  "gene_symbol": "PDE1A",
  "term_id": "GO:0141162",
  "gene_name": "Dual specificity calcium_calmodulin-dependent 3',5'-cyclic nucleotide phosphodiesterase 1A",
  "term_label": "negative regulation of cAMP/PKA signal transduction"
}